preQ1 synthase activity [GO:0033739] (molecular function) Relationships: is a type of oxidoreductase activity, acting on the CH-NH group of donors, NAD or NADP as acceptor [GO:0016646]; is_a oxidoreductase activity, acting on other nitrogenous compounds as donors, with NAD or NADP as acceptor [GO:0046857] Definition: Catalysis of the reaction: 7-aminomethyl-7-carbaguanine + 2 NADP+ = 7-cyano-7-deazaguanine + 2 NADPH + 3 H+. Sources: RHEA:13409 Also known as: 7-aminomethyl-7-carbaguanine:NADP+ oxidoreductase activity, 7-cyano-7-deazaguanine reductase activity, QueF, YkvM, preQ0 oxidoreductase activity, preQ0 reductase activity, queuine synthase activity, queuine:NADP+ oxidoreductase activity Note: Note that the reaction occurs in the reverse direction.